{
  "gene_symbol": "TMSB15B",
  "term_id": "GO:0030334",
  "gene_name": "Thymosin beta-15B",
  "term_label": "regulation of cell migration",
  "gene": "UniProtKB:P0CG35"
}